{
  "gene": "UniProtKB:Q92626",
  "gene_symbol": "PXDN",
  "term_id": "UNKNOWN:0002",
  "gene_name": "Peroxidasin homolog",
  "term_label": "Unknown biological process"
}